regulation of protein deneddylation [GO:0060625] (biological process) Sources: GOC:dph, GOC:tb Relationships: is a type of regulation of protein modification by small protein conjugation or removal [GO:1903320]; regulates protein deneddylation [GO:0000338] Definition: Any process that modulates the rate, frequency, or extent of protein deneddylation, the removal of a ubiquitin-like protein of the NEDD8 type from a protein. Also known as: regulation of cullin deneddylation